{
  "term_id": "GO:0005634",
  "gene_name": "Ubiquitin carboxyl-terminal hydrolase 17-like protein 21",
  "gene": "UniProtKB:D6R901",
  "term_label": "nucleus",
  "gene_symbol": "USP17L21"
}